positive regulation of serotonin uptake [GO:0051613] (biological process) Definition: Any process that activates or increases the frequency, rate or extent of the directed movement of serotonin into a cell. Relationships: is a type of positive regulation of neurotransmitter uptake [GO:0051582]; is a type of regulation of serotonin uptake [GO:0051611]; positively regulates serotonin uptake [GO:0051610] Also known as: positive regulation of 5-HT uptake, positive regulation of 5-hydroxytryptamine uptake, positive regulation of 5HT uptake, positive regulation of serotonin import, up regulation of serotonin uptake, up-regulation of serotonin uptake, upregulation of serotonin uptake, activation of serotonin uptake, stimulation of serotonin uptake Sources: GOC:ai